mitotic cleavage furrow ingression [GO:1990386] (biological process) Definition: Advancement of the mitotic cleavage furrow from the outside of the cell inward towards the center of the cell. The cleavage furrow acts as a 'purse string' which draws tight to separate daughter cells during mitotic cytokinesis and partition the cytoplasm between the two daughter cells. The furrow ingresses until a cytoplasmic bridge is formed. Relationships: is a type of cleavage furrow ingression [GO:0036090]; is a type of mitotic cytokinetic process [GO:1902410] References: PMID:12707312 Sources: GOC:kmv